{
  "gene_name": "Kremen protein 2",
  "gene": "UniProtKB:Q8NCW0",
  "gene_symbol": "KREMEN2",
  "term_label": "plasma membrane",
  "term_id": "GO:0005886"
}